{
  "gene_symbol": "GNG7",
  "term_label": "G protein-coupled receptor signaling pathway",
  "gene_name": "Guanine nucleotide-binding protein G(I)_G(S)_G(O) subunit gamma-7",
  "term_id": "GO:0007186",
  "gene": "UniProtKB:O60262"
}